{
  "gene_symbol": "ERAL1",
  "term_label": "mitochondrial matrix",
  "term_id": "GO:0005759",
  "gene_name": "GTPase Era, mitochondrial",
  "gene": "UniProtKB:O75616"
}